glycine receptor clustering [GO:0072579] (biological process) Definition: The receptor clustering process in which glycine receptors are localized to distinct domains in the cell membrane. Relationships: is a type of neurotransmitter-gated ion channel clustering [GO:0072578]; BFO_0000050 postsynaptic membrane organization [GO:0001941] References: PMID:20843816 Sources: GOC:dsf, GOC:mah, GOC:pr